neuron intrinsic apoptotic signaling pathway in response to endoplasmic reticulum stress [GO:0036483] (biological process) Regulation: RO_0002211 by regulation of endoplasmic reticulum stress-induced neuron intrinsic apoptotic signaling pathway [GO:1903381]; negatively regulated by negative regulation of endoplasmic reticulum stress-induced neuron intrinsic apoptotic signaling pathway [GO:1903382] Also known as: ER stress-induced neuron apoptosis, endoplasmic reticulum stress-induced neuron apoptosis, ER stress-induced neuron intrinsic apoptotic signaling pathway, endoplasmic reticulum stress-induced neuron intrinsic apoptotic signaling pathway Relationships: is a type of GO:0070059; is part of neuron apoptotic process [GO:0051402] Definition: The series of molecular signals in which an intracellular signal is conveyed to trigger the apoptotic death of a neuron. The pathway is induced in response to a stimulus indicating endoplasmic reticulum (ER) stress, and ends when the execution phase of apoptosis is triggered. ER stress usually results from the accumulation of unfolded or misfolded proteins in the ER lumen. References: PMID:21113145 Sources: GOC:PARL, GOC:bf